{
  "gene": "UniProtKB:P43681",
  "gene_symbol": "CHRNA4",
  "term_label": "membrane depolarization",
  "gene_name": "Neuronal acetylcholine receptor subunit alpha-4",
  "term_id": "GO:0051899"
}